{
  "term_label": "nucleic acid binding",
  "gene": "UniProtKB:Q99551",
  "gene_symbol": "MTERF1",
  "gene_name": "Transcription termination factor 1, mitochondrial",
  "term_id": "GO:0003676"
}